{
  "gene_name": "Matrix remodeling-associated protein 8",
  "term_id": "UNKNOWN:0001",
  "gene": "UniProtKB:Q9BRK3",
  "term_label": "Unknown molecular function",
  "gene_symbol": "MXRA8"
}